{
  "term_id": "GO:0048471",
  "term_label": "perinuclear region of cytoplasm",
  "gene_symbol": "EHD1",
  "gene_name": "EH domain-containing protein 1",
  "gene": "UniProtKB:Q9H4M9"
}